{
  "term_label": "cell surface receptor protein tyrosine kinase signaling pathway",
  "term_id": "GO:0007169",
  "gene_symbol": "RET",
  "gene_name": "Proto-oncogene tyrosine-protein kinase receptor Ret",
  "gene": "UniProtKB:P07949"
}